selenate adenylyltransferase (ATP) activity [GO:0098616] (molecular function) Definition: Catalysis of the reaction: ATP + H2SeO4 = diphosphate + adenylylselenate. References: PMID:2537056 Relationships: is a type of GO:0070566